regulation of L-tryptophan metabolic process [GO:0090357] (biological process) Sources: GOC:tb Definition: Any process that modulates the frequency, rate or extent of the chemical reactions and pathways involving tryptophan, the chiral amino acid 2-amino-3-(1H-indol-3-yl)propanoic acid. Also known as: regulation of tryptophan metabolism, regulation of tryptophan metabolic process Subtypes: positive regulation of L-tryptophan metabolic process [GO:0090358], GO:1901996, regulation of 'de novo' NAD biosynthetic process from L-tryptophan [GO:1905012] Relationships: is a type of regulation of amino acid metabolic process [GO:0006521]; is_a GO:0062012; regulates L-tryptophan metabolic process [GO:0006568]